{
  "term_id": "GO:0080025",
  "gene_symbol": "WIPI2",
  "term_label": "phosphatidylinositol-3,5-bisphosphate binding",
  "gene": "UniProtKB:Q9Y4P8",
  "gene_name": "WD repeat domain phosphoinositide-interacting protein 2"
}